{
  "gene_name": "Protein phosphatase 1 regulatory subunit 3G",
  "gene_symbol": "PPP1R3G",
  "term_label": "glycogen binding",
  "gene": "UniProtKB:B7ZBB8",
  "term_id": "GO:2001069"
}